{
  "term_label": "positive regulation of protein targeting to membrane",
  "gene_symbol": "C2CD5",
  "gene_name": "C2 domain-containing protein 5",
  "gene": "UniProtKB:Q86YS7",
  "term_id": "GO:0090314"
}